semaphorin-plexin signaling pathway involved in axon guidance [GO:1902287] (biological process) Also known as: semaphorin-plexin signaling pathway involved in axon pathfinding, semaphorin-plexin signalling pathway involved in axon guidance, semaphorin-plexin signalling pathway involved in axon pathfinding, semaphorin-plexin signaling pathway involved in axon growth cone guidance, semaphorin-plexin signalling pathway involved in axon growth cone guidance, semaphorin-plexin signaling pathway involved in axon chemotaxis, semaphorin-plexin signalling pathway involved in axon chemotaxis References: PMID:22790009 Sources: GOC:BHF, GOC:TermGenie, GOC:rl Definition: Any semaphorin-plexin signaling pathway that is involved in axon guidance. Relationships: is a type of GO:1902285; is part of axon guidance [GO:0007411]